glucan biosynthetic process [GO:0009250] (biological process) Sources: GOC:go_curators Subtypes: glycogen biosynthetic process [GO:0005978], GO:0009969, starch biosynthetic process [GO:0019252], GO:0030979, beta-glucan biosynthetic process [GO:0051274], pullulan biosynthetic process [GO:0051677], osmoregulated periplasmic glucan biosynthetic process [GO:1900727] Definition: The chemical reactions and pathways resulting in the formation of glucans, polysaccharides consisting only of glucose residues. Regulation: RO_0002211 by regulation of glucan biosynthetic process [GO:0010962] Also known as: glucan anabolism, glucan biosynthesis, glucan formation, glucan synthesis Relationships: is a type of polysaccharide biosynthetic process [GO:0000271]; is a type of GO:0044042